8-demethylnovobiocic acid C8-methyltransferase activity [GO:0102526] (MF) Definition: Catalysis of the reaction: S-adenosyl-L-methionine + 8-desmethylnovobiocic acid = S-adenosyl-L-homocysteine + novobiocic acid + H+. Sources: EC:2.1.1.284, GOC:pz Relationships: is a type of methyltransferase activity [GO:0008168]